L-galactose-1-phosphate phosphatase activity [GO:0010347] (molecular function) Relationships: is a type of galactose-1-phosphate phosphatase activity [GO:0070456] Definition: Catalysis of the reaction: L-galactose-1-phosphate + H2O = L-galactose + phosphate. References: PMID:15550539, PMID:16595667